{
  "gene_symbol": "ISG20",
  "term_label": "negative regulation of viral genome replication",
  "term_id": "GO:0045071",
  "gene_name": "Interferon-stimulated gene 20 kDa protein",
  "gene": "UniProtKB:Q96AZ6"
}